{
  "gene_symbol": "WIZ",
  "gene_name": "Protein Wiz",
  "term_label": "RNA polymerase II cis-regulatory region sequence-specific DNA binding",
  "term_id": "GO:0000978",
  "gene": "UniProtKB:O95785"
}